negative regulation of anion transmembrane transport [GO:1903960] (biological process) Relationships: is_a negative regulation of monoatomic ion transmembrane transport [GO:0034766]; is a type of GO:1903792; is a type of regulation of monoatomic anion transmembrane transport [GO:1903959]; negatively regulates GO:0098656 Subtypes: GO:0010360, negative regulation of iodide transmembrane transport [GO:1904213] Also known as: down regulation of anion transmembrane transport, down-regulation of anion transmembrane transport, downregulation of anion transmembrane transport, inhibition of anion transmembrane transport Definition: Any process that stops, prevents or reduces the frequency, rate or extent of anion transmembrane transport. Sources: GOC:TermGenie, GOC:vw, GO_REF:0000058